{
  "term_label": "cytoplasmic side of late endosome membrane",
  "gene": "UniProtKB:Q9H305",
  "term_id": "GO:0098560",
  "gene_name": "Cell death-inducing p53-target protein 1",
  "gene_symbol": "CDIP1"
}